TIRAP-dependent toll-like receptor signaling pathway [GO:0035664] (biological process) Definition: The series of molecular signals initiated by a ligand binding to a toll-like receptor where the TIRAP/MAL adaptor mediates transduction of the signal. Toll-like receptors directly bind pattern motifs from a variety of microbial sources to initiate an innate immune response. Subtypes: TIRAP-dependent toll-like receptor 4 signaling pathway [GO:0035665] Relationships: is a type of toll-like receptor signaling pathway [GO:0002224] Also known as: MAL-dependent toll-like receptor signaling pathway, MyD88 adapter-like dependent toll-like receptor signaling pathway, TIRAP-dependent TLR signaling pathway, TIRAP-dependent toll-like receptor signalling pathway References: PMID:11526399, PMID:11544529, PMID:12447442 Sources: GOC:BHF